positive regulation of the force of heart contraction by norepinephrine [GO:0003061] (biological process) Definition: The process in which the secretion of norepinephrine into the bloodstream or released from nerve endings modulates the force of heart musclecontraction. Relationships: is a type of positive regulation of the force of heart contraction by chemical signal [GO:0003099]; BFO_0000050 positive regulation of the force of heart contraction by epinephrine-norepinephrine [GO:0001997] Sources: GOC:mtg_cardio, GOC:rl Subtypes: positive regulation of the force of heart contraction by circulating norepinephrine [GO:0003109], positive regulation of the force of heart contraction by neuronal norepinephrine [GO:0003110] Also known as: increased force of heart contraction by norepinephrine, noradrenaline cardiac inotropy, noradrenaline regulation of the strength of heart muscle contraction, norepinephrine cardiac inotropy, increased force of heart contraction by adrenaline, positive regulation of heart contraction by adrenaline, positive regulation of heart contraction by norepinephrine